{
  "gene_name": "Putative uncharacterized protein LOC642776",
  "term_label": "Unknown biological process",
  "gene_symbol": "Q9BTK2",
  "term_id": "UNKNOWN:0002",
  "gene": "UniProtKB:Q9BTK2"
}